{
  "term_label": "protein K48-linked ubiquitination",
  "gene_name": "F-box only protein 38",
  "gene": "UniProtKB:Q6PIJ6",
  "gene_symbol": "FBXO38",
  "term_id": "GO:0070936"
}